{
  "term_label": "Unknown molecular function",
  "gene_name": "Testis-specific gene 13 protein",
  "gene": "UniProtKB:Q96PP4",
  "gene_symbol": "TSGA13",
  "term_id": "UNKNOWN:0001"
}